{
  "gene": "UniProtKB:P50406",
  "gene_symbol": "HTR6",
  "term_label": "neurotransmitter receptor activity",
  "term_id": "GO:0030594",
  "gene_name": "5-hydroxytryptamine receptor 6"
}